{
  "term_id": "GO:0003677",
  "gene": "UniProtKB:Q8TDI0",
  "term_label": "DNA binding",
  "gene_name": "Chromodomain-helicase-DNA-binding protein 5",
  "gene_symbol": "CHD5"
}